negative regulation of macrophage antigen processing and presentation [GO:0002617] (biological process) Also known as: down regulation of macrophage antigen processing and presentation, down-regulation of macrophage antigen processing and presentation, downregulation of macrophage antigen processing and presentation, inhibition of macrophage antigen processing and presentation Definition: Any process that stops, prevents, or reduces the frequency, rate, or extent of macrophage antigen processing and presentation. Sources: GOC:add Relationships: is a type of negative regulation of antigen processing and presentation [GO:0002578]; is a type of regulation of macrophage antigen processing and presentation [GO:0002616]; negatively regulates GO:0002472